{
  "term_label": "peptide receptor activity",
  "gene_symbol": "NPR1",
  "gene_name": "Atrial natriuretic peptide receptor 1",
  "gene": "UniProtKB:P16066",
  "term_id": "GO:0001653"
}